{
  "term_id": "GO:0098971",
  "term_label": "anterograde dendritic transport of neurotransmitter receptor complex",
  "gene_symbol": "KIF17",
  "gene": "UniProtKB:Q9P2E2",
  "gene_name": "Kinesin-like protein KIF17"
}